{
  "gene_name": "Rod cGMP-specific 3',5'-cyclic phosphodiesterase subunit alpha",
  "term_label": "retina development in camera-type eye",
  "gene_symbol": "PDE6A",
  "term_id": "GO:0060041",
  "gene": "UniProtKB:P16499"
}